outer acrosomal membrane [GO:0002081] (cellular component) Note: Note that this term is not a descendant of 'organelle outer membrane ; GO:0031968' because the outer acrosomal membrane is a portion of the acrosomal membrane; the latter is a single lipid bilayer. References: PMID:8936405 Sources: GOC:dph Relationships: is a type of cytoplasmic vesicle membrane [GO:0030659]; is part of acrosomal membrane [GO:0002080] Definition: The acrosomal membrane region that underlies the plasma membrane of the sperm. This membrane fuses with the sperm plasma membrane as part of the acrosome reaction.